cell-cell signaling involved in kidney development [GO:0060995] (biological process) Subtypes: cell-cell signaling involved in pronephros development [GO:0039016], cell-cell signaling involved in mesonephros development [GO:0061210], cell-cell signaling involved in metanephros development [GO:0072204] Also known as: cell-cell signalling involved in kidney development Sources: GOC:dph, GOC:mtg_kidney_jan10 Definition: Any process that mediates the transfer of information from one cell to another and contributes to the progression of the kidney over time, from its formation to the mature organ. Relationships: is a type of cell-cell signaling [GO:0007267]; is part of kidney development [GO:0001822]